positive regulation of protein localization to adherens junction [GO:1904704] (biological process) Definition: Any process that activates or increases the frequency, rate or extent of protein localization to adherens junction. An adherens junction is a cell-cell junction composed of the epithelial cadherin-catenin complex at which the cytoplasmic face of the plasma membrane is attached to actin filaments. References: PMID:26412237 Sources: GOC:TermGenie, GOC:aruk, GOC:bc, GOC:kmv, GO_REF:0000058 Relationships: is a type of positive regulation of protein localization to cell-cell junction [GO:0150107]; is a type of GO:1904702; positively regulates GO:0071896 Also known as: positive regulation of protein localisation in cell-cell adherens junction, positive regulation of protein localisation to cell-cell adherens junction, positive regulation of protein localization in cell-cell adherens junction, up regulation of protein localisation in cell-cell adherens junction, up regulation of protein localisation to cell-cell adherens junction, up regulation of protein localization in cell-cell adherens junction, up regulation of protein localization to cell-cell adherens junction, up-regulation of protein localisation in cell-cell adherens junction, up-regulation of protein localisation to cell-cell adherens junction, up-regulation of protein localization in cell-cell adherens junction, up-regulation of protein localization to cell-cell adherens junction, upregulation of protein localisation in cell-cell adherens junction, upregulation of protein localisation to cell-cell adherens junction, upregulation of protein localization in cell-cell adherens junction, upregulation of protein localization to cell-cell adherens junction, activation of protein localisation in cell-cell adherens junction, activation of protein localisation to cell-cell adherens junction, activation of protein localization in cell-cell adherens junction, activation of protein localization to cell-cell adherens junction